{
  "gene_name": "Tenascin-N",
  "term_id": "GO:0005178",
  "gene": "UniProtKB:Q9UQP3",
  "term_label": "integrin binding",
  "gene_symbol": "TNN"
}